D-galactonate transmembrane transport [GO:0042875] (biological process) Also known as: D-galactonate transport Sources: GOC:jl, GOC:jsg, GOC:mah Relationships: is a type of carbohydrate transmembrane transport [GO:0034219]; is a type of aldonate transmembrane transport [GO:0042873] Definition: The process in which D-galactonate, the D-enantiomer of galactonate, is transported across a lipid bilayer, from one side of a membrane to the other.